{
  "gene": "UniProtKB:Q9NVE7",
  "term_label": "nucleus",
  "gene_name": "4'-phosphopantetheine phosphatase",
  "term_id": "GO:0005634",
  "gene_symbol": "PANK4"
}